{
  "term_id": "GO:0005634",
  "gene_name": "Centromere protein F",
  "term_label": "nucleus",
  "gene": "UniProtKB:P49454",
  "gene_symbol": "CENPF"
}